pentalenene synthase activity [GO:0050467] (molecular function) Relationships: is a type of GO:0010334 Also known as: 2-trans,6-trans-farnesyl-diphosphate diphosphate-lyase (cyclizing, pentalenene-forming), 2-trans,6-trans-farnesyldiphosphate diphosphate-lyase (cyclizing, pentalenene-forming), pentalenene synthetase activity Definition: Catalysis of the reaction: 2-trans,6-trans-farnesyl diphosphate = diphosphate + pentalenene. Sources: EC:4.2.3.7, RHEA:18081